{
  "gene_symbol": "CCDC185",
  "gene_name": "Coiled-coil domain-containing protein 185",
  "gene": "UniProtKB:Q8N715",
  "term_id": "UNKNOWN:0003",
  "term_label": "Unknown cellular component"
}